{
  "gene_symbol": "PPP2R3A",
  "gene": "UniProtKB:Q06190",
  "gene_name": "Serine_threonine-protein phosphatase 2A regulatory subunit B'' subunit alpha",
  "term_label": "somatic muscle development",
  "term_id": "GO:0007525"
}